ubiquinol:oxygen oxidoreductase activity [GO:0102721] (molecular function) Definition: Catalysis of the reaction: O2 + 2 an ubiquinol = 2 H2O + 2 an ubiquinone. Sources: GOC:pz, RHEA:30255 Relationships: is a type of oxidoreductase activity, acting on diphenols and related substances as donors, oxygen as acceptor [GO:0016682]